sodium:sulfate symporter activity [GO:0015382] (MF) Relationships: is a type of secondary active sulfate transmembrane transporter activity [GO:0008271]; is a type of GO:0015370 Sources: TC:2.A.47.1.2 Definition: Enables the transfer of a solute or solutes from one side of a membrane to the other according to the reaction: sulfate(out) + Na+(out) = sulfate(in) + Na+(in). Also known as: sodium:sulfate cotransporter activity, sodium:sulphate symporter activity